{
  "gene_symbol": "NUAK1",
  "term_id": "GO:0004674",
  "gene_name": "NUAK family SNF1-like kinase 1",
  "gene": "UniProtKB:O60285",
  "term_label": "protein serine/threonine kinase activity"
}